positive regulation of leukocyte adhesion to arterial endothelial cell [GO:1904999] (biological process) Relationships: is_a positive regulation of leukocyte adhesion to vascular endothelial cell [GO:1904996]; is a type of regulation of leukocyte adhesion to arterial endothelial cell [GO:1904997]; positively regulates GO:0061757 Also known as: up regulation of leukocyte adhesion to arterial endothelial cell, up-regulation of leukocyte adhesion to arterial endothelial cell, upregulation of leukocyte adhesion to arterial endothelial cell, activation of leukocyte adhesion to arterial endothelial cell References: PMID:22267480 Sources: GOC:BHF, GOC:BHF_miRNA, GOC:TermGenie, GOC:bc, GO_REF:0000058 Definition: Any process that activates or increases the frequency, rate or extent of leukocyte adhesion to arterial endothelial cell.